{
  "gene_symbol": "CD300LD-AS1",
  "gene_name": "Uncharacterized protein CD300LD-AS1",
  "term_label": "Unknown molecular function",
  "term_id": "UNKNOWN:0001",
  "gene": "UniProtKB:Q96MU5"
}